{
  "term_id": "GO:0005829",
  "gene_name": "Serine_threonine-protein phosphatase 6 regulatory subunit 2",
  "term_label": "cytosol",
  "gene_symbol": "PPP6R2",
  "gene": "UniProtKB:O75170"
}